internal mRNA (guanine-N7-)-methyltransferase activity [GO:0160090] (molecular function) Definition: Catalysis of the reaction: a guanosine in mRNA + S-adenosyl-L-methionine = an N(7)-methylguanosine in mRNA + S-adenosyl-L-homocysteine. Relationships: is a type of mRNA methyltransferase activity [GO:0008174]; is part of RNA (guanine-N7)-methylation [GO:0036265] References: PMID:31031084, PMID:37379838 Sources: RHEA:60508